{
  "gene": "UniProtKB:Q9NZB2",
  "term_id": "UNKNOWN:0001",
  "gene_symbol": "FAM120A",
  "term_label": "Unknown molecular function",
  "gene_name": "Constitutive coactivator of PPAR-gamma-like protein 1"
}